{
  "term_id": "GO:0042393",
  "gene_name": "Protein SETSIP",
  "gene": "UniProtKB:P0DME0",
  "gene_symbol": "SETSIP",
  "term_label": "histone binding"
}